death receptor agonist activity [GO:0038177] (MF) Also known as: death receptor activator activity Definition: Interacting with a death receptor such that the proportion of death receptors in an active form is increased. Ligand binding to a death receptor often induces a conformational change to activate the receptor. Relationships: is a type of GO:0048018; has part death receptor binding [GO:0005123]; positively regulates GO:0005035 Sources: GOC:mtg_apoptosis, GOC:pr